{
  "gene_symbol": "ARHGEF12",
  "gene_name": "Rho guanine nucleotide exchange factor 12",
  "term_id": "GO:0005737",
  "term_label": "cytoplasm",
  "gene": "UniProtKB:Q9NZN5"
}